{
  "gene_name": "Interferon-induced transmembrane protein 5",
  "gene_symbol": "IFITM5",
  "term_label": "bone mineralization",
  "term_id": "GO:0030282",
  "gene": "UniProtKB:A6NNB3"
}